protein localization to lysosome [GO:0061462] (biological process) Regulation: regulated by GO:0150031; positively regulated by GO:0150032; negatively regulated by negative regulation of protein localization to lysosome [GO:0150033] Definition: A process in which a protein is transported to, or maintained in, a location within a lysosome. Subtypes: protein targeting to lysosome [GO:0006622], GO:0098943 Relationships: is_a protein localization to vacuole [GO:0072665] Sources: GOC:dph